positive regulation of pancreatic amylase secretion [GO:1902278] (biological process) Definition: Any process that activates or increases the frequency, rate or extent of pancreatic amylase secretion. References: PMID:19028687 Sources: GOC:TermGenie, GOC:jc Relationships: is a type of positive regulation of protein secretion [GO:0050714]; is a type of regulation of pancreatic amylase secretion [GO:1902276]; positively regulates pancreatic amylase secretion [GO:0036395] Subtypes: GO:1902279 Also known as: up regulation of pancreatic amylase secretion, up-regulation of pancreatic amylase secretion, upregulation of pancreatic amylase secretion, activation of pancreatic amylase secretion